{
  "gene_name": "Lutropin-choriogonadotropic hormone receptor",
  "term_label": "ovarian follicle development",
  "gene": "UniProtKB:P22888",
  "term_id": "GO:0001541",
  "gene_symbol": "LHCGR"
}